{
  "term_label": "regulation of transcription by RNA polymerase II",
  "term_id": "GO:0006357",
  "gene": "UniProtKB:P52952",
  "gene_name": "Homeobox protein Nkx-2.5",
  "gene_symbol": "NKX2-5"
}